signal transduction by p53 class mediator [GO:0072331] (biological process) Subtypes: DNA damage response, signal transduction by p53 class mediator [GO:0030330], GO:0072332 Definition: An intracellular signaling process that is induced by the cell cycle regulator phosphoprotein p53 or an equivalent protein. Relationships: is a type of intracellular signal transduction [GO:0035556] Sources: GOC:mah Regulation: regulated by GO:1901796; negatively regulated by negative regulation of signal transduction by p53 class mediator [GO:1901797]; positively regulated by positive regulation of signal transduction by p53 class mediator [GO:1901798]